{
  "term_label": "lysosomal transport",
  "gene": "UniProtKB:Q68CP4",
  "gene_name": "Heparan-alpha-glucosaminide N-acetyltransferase",
  "gene_symbol": "HGSNAT",
  "term_id": "GO:0007041"
}